{
  "term_label": "cellular response to hormone stimulus",
  "gene_symbol": "NCOA3",
  "gene_name": "Nuclear receptor coactivator 3",
  "gene": "UniProtKB:Q9Y6Q9",
  "term_id": "GO:0032870"
}